{
  "gene_symbol": "TSHZ2",
  "gene": "UniProtKB:Q9NRE2",
  "term_id": "GO:0006357",
  "gene_name": "Teashirt homolog 2",
  "term_label": "regulation of transcription by RNA polymerase II"
}